{
  "term_id": "GO:0005675",
  "term_label": "transcription factor TFIIH holo complex",
  "gene_symbol": "GTF2H1",
  "gene_name": "General transcription factor IIH subunit 1",
  "gene": "UniProtKB:P32780"
}